{
  "gene_symbol": "NLRP7",
  "gene_name": "NACHT, LRR and PYD domains-containing protein 7",
  "gene": "UniProtKB:Q8WX94",
  "term_id": "GO:0005737",
  "term_label": "cytoplasm"
}